{
  "gene_name": "HLA class I histocompatibility antigen, alpha chain G",
  "gene_symbol": "HLA-G",
  "term_label": "positive regulation of T cell mediated cytotoxicity",
  "gene": "UniProtKB:P17693",
  "term_id": "GO:0001916"
}